{
  "term_id": "UNKNOWN:0003",
  "gene_name": "Chymotrypsin-C",
  "term_label": "Unknown cellular component",
  "gene": "UniProtKB:Q99895",
  "gene_symbol": "CTRC"
}